{
  "gene": "UniProtKB:Q9UHJ3",
  "gene_name": "Scm-like with four MBT domains protein 1",
  "term_label": "chromatin binding",
  "term_id": "GO:0003682",
  "gene_symbol": "SFMBT1"
}